{
  "term_label": "cytoplasm",
  "gene_symbol": "PLEKHH2",
  "gene_name": "Pleckstrin homology domain-containing family H member 2",
  "term_id": "GO:0005737",
  "gene": "UniProtKB:Q8IVE3"
}